{
  "gene_name": "Pleckstrin homology domain-containing family A member 3",
  "gene": "UniProtKB:Q9HB20",
  "term_id": "GO:0055037",
  "gene_symbol": "PLEKHA3",
  "term_label": "recycling endosome"
}